{
  "gene_symbol": "TBX22",
  "term_label": "nucleus",
  "gene_name": "T-box transcription factor TBX22",
  "gene": "UniProtKB:Q9Y458",
  "term_id": "GO:0005634"
}